{
  "gene": "UniProtKB:P18545",
  "term_label": "photoreceptor outer segment membrane",
  "gene_name": "Retinal rod rhodopsin-sensitive cGMP 3',5'-cyclic phosphodiesterase subunit gamma",
  "term_id": "GO:0042622",
  "gene_symbol": "PDE6G"
}